{
  "term_id": "GO:0005737",
  "gene_symbol": "PKIG",
  "gene": "UniProtKB:Q9Y2B9",
  "term_label": "cytoplasm",
  "gene_name": "cAMP-dependent protein kinase inhibitor gamma"
}